polarized secretion of basement membrane proteins in epithelium [GO:0061865] (BP) References: PMID:26610918, PMID:28228250 Definition: The basement membrane constituent secretion in which there is a restriction or targeting of basement membrane proteins for controlled release on the basal side of polarized epithelium. Relationships: is a type of GO:0061864